enone reductase activity [GO:0035671] (molecular function) Definition: Catalysis of the reaction: an enone + NADPH + H+ = a ketone + NADP+. References: PMID:17945329, PMID:19166903 Sources: GOC:kad Relationships: is a type of oxidoreductase activity, acting on the CH-CH group of donors, NAD or NADP as acceptor [GO:0016628] Subtypes: 3-oxo-5-alpha-steroid 4-dehydrogenase (NADP+) activity [GO:0047751], GO:0047787, GO:0052581